positive regulation of cellular response to macrophage colony-stimulating factor stimulus [GO:1903974] (BP) Relationships: is a type of GO:1903971; is a type of regulation of cellular response to macrophage colony-stimulating factor stimulus [GO:1903972]; positively regulates cellular response to macrophage colony-stimulating factor stimulus [GO:0036006] Also known as: positive regulation of cellular response to M-CSF stimulus, positive regulation of cellular response to macrophage colony-stimulating factor, up regulation of cellular response to M-CSF stimulus, up regulation of cellular response to macrophage colony-stimulating factor, up regulation of cellular response to macrophage colony-stimulating factor stimulus, up-regulation of cellular response to M-CSF stimulus, up-regulation of cellular response to macrophage colony-stimulating factor, up-regulation of cellular response to macrophage colony-stimulating factor stimulus, upregulation of cellular response to M-CSF stimulus, upregulation of cellular response to macrophage colony-stimulating factor, upregulation of cellular response to macrophage colony-stimulating factor stimulus, activation of cellular response to M-CSF stimulus, activation of cellular response to macrophage colony-stimulating factor, activation of cellular response to macrophage colony-stimulating factor stimulus Definition: Any process that activates or increases the frequency, rate or extent of cellular response to macrophage colony-stimulating factor stimulus. References: PMID:19100238 Sources: GOC:BHF, GOC:TermGenie, GOC:nc, GO_REF:0000058